negative regulation of DNA recombination at centromere [GO:0061808] (biological process) Also known as: negative regulation of centromeric recombination Definition: Any process that stops, prevents, or reduces the frequency, rate or extent of genetic recombination at the centromere. Relationships: is a type of negative regulation of DNA recombination [GO:0045910]; is a type of regulation of DNA recombination at centromere [GO:0061806] Sources: GOC:dph, GOC:mah